{
  "term_id": "GO:0005634",
  "gene_name": "Putative RRN3-like protein RRN3P2",
  "term_label": "nucleus",
  "gene_symbol": "RRN3P2",
  "gene": "UniProtKB:A6NIE6"
}